{
  "gene_symbol": "UBE2O",
  "term_id": "GO:0042147",
  "gene_name": "(E3-independent) E2 ubiquitin-conjugating enzyme",
  "term_label": "retrograde transport, endosome to Golgi",
  "gene": "UniProtKB:Q9C0C9"
}